euchromatin binding [GO:1990188] (molecular function) Definition: Binding to euchromatin, a dispersed and relatively uncompacted form of chromatin. References: PMID:22431512 Sources: GOC:vw Relationships: is a type of chromatin binding [GO:0003682]